{
  "gene_symbol": "TJAP1",
  "term_label": "trans-Golgi network",
  "gene": "UniProtKB:Q5JTD0",
  "term_id": "GO:0005802",
  "gene_name": "Tight junction-associated protein 1"
}